protein S-linked glycosylation [GO:0018280] (biological process) Definition: A protein glycosylation process in which a carbohydrate or carbohydrate derivative unit is added to a protein via a sulfur atom of a peptidyl-amino-acid such as cysteine or methionine. Sources: GOC:ai, GOC:jsg, GOC:pr Relationships: is_a glycoprotein biosynthetic process [GO:0009101] Also known as: protein amino acid S-linked glycosylation